microtubule organizing center attachment site organization [GO:0034994] (biological process) Definition: A process that is carried out at the cellular level which results in the assembly, arrangement of constituent parts, or disassembly of a microtubule organizing center attachment site. A microtubule organizing center attachment site is a region of the nuclear envelope to which a microtubule organizing center (MTOC) attaches. Relationships: is a type of cellular component organization [GO:0016043]; is part of GO:0006998 References: PMID:18692466 Sources: GOC:mah Also known as: MAS organization, MTOC attachment site organization, microtubule organising centre attachment site organisation